cellular response to proline [GO:0071235] (biological process) Relationships: is a type of GO:0010238; is a type of cellular response to amino acid stimulus [GO:0071230]; is a type of cellular response to nitrogen compound [GO:1901699]; is a type of cellular response to oxygen-containing compound [GO:1901701] Definition: Any process that results in a change in state or activity of a cell (in terms of movement, secretion, enzyme production, gene expression, etc.) as a result of a proline stimulus. Sources: GOC:mah